{
  "term_id": "GO:0006508",
  "gene_symbol": "PGC",
  "gene": "UniProtKB:P20142",
  "gene_name": "Gastricsin",
  "term_label": "proteolysis"
}